L-arabinose transmembrane transport [GO:0042882] (biological process) Relationships: is a type of arabinose transmembrane transport [GO:0015751] Definition: The process in which L-arabinose, the L-enantiomer of arabinose, is transported across a lipid bilayer, from one side of a membrane to the other. Sources: GOC:jl, GOC:jsg, GOC:mah, ISBN:0198506732 Also known as: L-arabinose transport